{
  "gene_name": "DEP domain-containing mTOR-interacting protein",
  "gene": "UniProtKB:Q8TB45",
  "gene_symbol": "DEPTOR",
  "term_id": "GO:0030291",
  "term_label": "protein serine/threonine kinase inhibitor activity"
}